{
  "gene_symbol": "TUBA1B",
  "term_id": "GO:0030182",
  "gene_name": "Tubulin alpha-1B chain",
  "term_label": "neuron differentiation",
  "gene": "UniProtKB:P68363"
}